{
  "gene": "UniProtKB:O00567",
  "term_label": "small-subunit processome",
  "gene_name": "Nucleolar protein 56",
  "term_id": "GO:0032040",
  "gene_symbol": "NOP56"
}